regulation of receptor internalization [GO:0002090] (biological process) Relationships: is a type of regulation of receptor-mediated endocytosis [GO:0048259]; regulates receptor internalization [GO:0031623] Subtypes: negative regulation of receptor internalization [GO:0002091], positive regulation of receptor internalization [GO:0002092], regulation of postsynaptic neurotransmitter receptor internalization [GO:0099149], regulation of G protein-coupled receptor internalization [GO:1904020] Definition: Any process that modulates the frequency, rate or extent of receptor internalization. Sources: GOC:hjd